{
  "term_label": "Unknown biological process",
  "gene": "UniProtKB:O96005",
  "term_id": "UNKNOWN:0002",
  "gene_symbol": "CLPTM1",
  "gene_name": "Putative lipid scramblase CLPTM1"
}